{
  "gene": "UniProtKB:Q99542",
  "gene_name": "Matrix metalloproteinase-19",
  "gene_symbol": "MMP19",
  "term_id": "GO:0030198",
  "term_label": "extracellular matrix organization"
}